{
  "gene": "UniProtKB:O60229",
  "gene_name": "Kalirin",
  "term_label": "extrinsic component of membrane",
  "gene_symbol": "KALRN",
  "term_id": "GO:0019898"
}